beta-ketoacyl-acyl-carrier-protein synthase III activity [GO:0033818] (molecular function) Sources: EC:2.3.1.180 Relationships: is a type of GO:0016747 Also known as: 3-ketoacyl-acyl carrier protein synthase III activity, 3-oxoacyl:ACP synthase III activity, FabH, KAS III, KASIII, acetyl-CoA:malonyl-acyl-carrier-protein C-acyltransferase activity, beta-ketoacyl (acyl carrier protein) synthase III activity, beta-ketoacyl-ACP synthase III activity, beta-ketoacyl-acyl carrier protein synthase III activity Definition: Catalysis of the reaction: acetyl-CoA + malonyl-[acyl-carrier protein] = acetoacyl-[acyl-carrier protein] + CoA + CO2.